{
  "gene": "UniProtKB:A0A075B710",
  "term_id": "UNKNOWN:0003",
  "term_label": "Unknown cellular component",
  "gene_name": "T cell receptor alpha joining 39 (Fragment)",
  "gene_symbol": "TRAJ39"
}